3-deoxy-7-phosphoheptulonate synthase activity [GO:0003849] (molecular function) Definition: Catalysis of the reaction: D-erythrose 4-phosphate + H2O + phosphoenolpyruvate = 7-phospho-2-dehydro-3-deoxy-D-arabino-heptonate + phosphate. Relationships: is a type of transferase activity, transferring alkyl or aryl (other than methyl) groups [GO:0016765] Sources: EC:2.5.1.54, RHEA:14717 Also known as: 2-dehydro-3-deoxyphosphoheptonate aldolase activity, 2-dehydro-3-deoxy-phosphoheptonate aldolase activity, 2-keto-3-deoxy-D-arabino-heptonic acid 7-phosphate synthetase activity, 3-deoxy-D-arabino-2-heptulosonic acid 7-phosphate synthetase activity, 3-deoxy-D-arabino-heptolosonate-7-phosphate synthetase activity, 3-deoxy-D-arabino-heptulosonate 7-phosphate synthetase activity, 7-phospho-2-dehydro-3-deoxy-D-arabino-heptonate, 7-phospho-2-dehydro-3-deoxy-D-arabino-heptonate D-erythrose-4-phosphate lyase (pyruvate-phosphorylating) activity, 7-phospho-2-keto-3-deoxy-D-arabino-heptonate D-erythrose-4-phosphate lyase (pyruvate-phosphorylating) activity, D-erythrose-4-phosphate-lyase (pyruvate-phosphorylating) activity, D-erythrose-4-phosphate-lyase activity, DAH7-P synthase activity, DAHP synthase activity, DHAP synthase activity, DS-Co activity, DS-Mn activity, KDPH synthase activity, KDPH synthetase activity, deoxy-D-arabino-heptulosonate-7-phosphate synthetase activity, phospho-2-dehydro-3-deoxyheptonate aldolase activity, phospho-2-keto-3-deoxyheptanoate aldolase activity, phospho-2-keto-3-deoxyheptonate aldolase activity, phospho-2-keto-3-deoxyheptonic aldolase activity, phospho-2-oxo-3-deoxyheptonate aldolase activity, phosphoenolpyruvate:D-erythrose-4-phosphate C-(1-carboxyvinyl)transferase (phosphate-hydrolysing, 2-carboxy-2-oxoethyl-forming)